chloride channel activity [GO:0005254] (molecular function) Subtypes: intracellularly calcium-gated chloride channel activity [GO:0005229], voltage-gated chloride channel activity [GO:0005247], GO:0005260, extracellularly glutamate-gated chloride channel activity [GO:0008068], GO:0016934, histamine-gated chloride channel activity [GO:0019182], GO:0022851, glycine-gated chloride ion channel activity [GO:0022852], pH-gated chloride channel activity [GO:0061797], volume-sensitive chloride channel activity [GO:0072320], serotonin-gated chloride channel activity [GO:0160039] Sources: GOC:mtg_transport, GOC:pr, ISBN:0815340729 Relationships: is a type of monoatomic anion channel activity [GO:0005253]; is a type of chloride transmembrane transporter activity [GO:0015108] Definition: Enables the energy-independent facilitated diffusion of a chloride ion through a transmembrane aqueous pore or channel. Regulation: regulated by chloride channel regulator activity [GO:0017081]; negatively regulated by chloride channel inhibitor activity [GO:0019869]